{
  "term_label": "Unknown molecular function",
  "gene": "UniProtKB:Q96DN0",
  "gene_symbol": "ERP27",
  "term_id": "UNKNOWN:0001",
  "gene_name": "Endoplasmic reticulum resident protein 27"
}